{
  "term_label": "actin filament organization",
  "term_id": "GO:0007015",
  "gene": "UniProtKB:P37802",
  "gene_symbol": "TAGLN2",
  "gene_name": "Transgelin-2"
}